{
  "gene": "UniProtKB:Q15596",
  "gene_name": "Nuclear receptor coactivator 2",
  "term_label": "positive regulation of transcription by RNA polymerase II",
  "gene_symbol": "NCOA2",
  "term_id": "GO:0045944"
}